{
  "gene": "UniProtKB:Q9NPJ1",
  "term_label": "kinociliary basal body",
  "term_id": "GO:1902636",
  "gene_symbol": "MKKS",
  "gene_name": "Molecular chaperone MKKS"
}